{
  "gene": "UniProtKB:Q9HAK2",
  "gene_symbol": "EBF2",
  "term_label": "regulation of transcription by RNA polymerase II",
  "gene_name": "Transcription factor COE2",
  "term_id": "GO:0006357"
}